{
  "term_id": "GO:0097730",
  "gene_name": "Intraflagellar transport protein 122 homolog",
  "gene_symbol": "IFT122",
  "term_label": "non-motile cilium",
  "gene": "UniProtKB:Q9HBG6"
}